{
  "gene_symbol": "KIF2A",
  "term_id": "GO:0003777",
  "gene_name": "Kinesin-like protein KIF2A",
  "term_label": "microtubule motor activity",
  "gene": "UniProtKB:O00139"
}